{
  "gene": "UniProtKB:Q8N808",
  "term_id": "GO:0016020",
  "term_label": "membrane",
  "gene_symbol": "SLC35G3",
  "gene_name": "Solute carrier family 35 member G3"
}